{
  "gene_symbol": "EGR1",
  "gene": "UniProtKB:P18146",
  "gene_name": "Early growth response protein 1",
  "term_label": "RNA polymerase II cis-regulatory region sequence-specific DNA binding",
  "term_id": "GO:0000978"
}